cyanidin 3-O-glucoside 2-O-glucuronosyltransferase activity [GO:0102160] (molecular function) Also known as: cyanidin-3-O-glucoside 2-O-glucuronosyltransferase activity Definition: Catalysis of the reaction: cyanidin 3-O-beta-D-glucoside betaine + UDP-alpha-D-glucuronate = H+ + cyanidin 3-O-beta-(2-O-beta-D-glucuronosyl)-beta-D-glucoside + UDP. Relationships: is a type of hexosyltransferase activity [GO:0016758] Sources: RHEA:28258